regulation of kidney development [GO:0090183] (biological process) Subtypes: GO:0061217, GO:0072215, positive regulation of kidney development [GO:0090184], negative regulation of kidney development [GO:0090185], regulation of branching involved in ureteric bud morphogenesis [GO:0090189], regulation of glomerulus development [GO:0090192] Relationships: is a type of GO:0050793; regulates kidney development [GO:0001822] Definition: Any process that modulates the rate, frequency or extent of kidney development. Kidney development is the process whose specific outcome is the progression of the kidney over time, from its formation to the mature structure. The kidney is an organ that filters the blood and excretes the end products of body metabolism in the form of urine. Sources: GOC:dph, GOC:tb, GOC:yaf Also known as: regulation of nephrogenesis